{
  "term_id": "GO:0030277",
  "gene_symbol": "TFF2",
  "term_label": "maintenance of gastrointestinal epithelium",
  "gene": "UniProtKB:Q03403",
  "gene_name": "Trefoil factor 2"
}